{
  "gene_name": "Thiol S-methyltransferase TMT1B",
  "term_label": "thiol S-methyltransferase activity",
  "gene_symbol": "TMT1B",
  "term_id": "GO:0018708",
  "gene": "UniProtKB:Q6UX53"
}